negative regulation of transforming growth factor beta3 production [GO:0032913] (biological process) Definition: Any process that stops, prevents, or reduces the frequency, rate, or extent of production of transforming growth factor-beta3. Also known as: down regulation of transforming growth factor-beta3 production, down-regulation of transforming growth factor-beta3 production, downregulation of transforming growth factor-beta3 production, negative regulation of TGF-B3 production, negative regulation of TGFB3 production, negative regulation of transforming growth factor-beta3 production, inhibition of transforming growth factor-beta3 production Relationships: is a type of regulation of transforming growth factor beta3 production [GO:0032910]; is_a GO:0071635; negatively regulates GO:0032907 Sources: GOC:mah